{
  "term_id": "GO:0002025",
  "term_label": "norepinephrine-epinephrine-mediated vasodilation involved in regulation of systemic arterial blood pressure",
  "gene_name": "Beta-1 adrenergic receptor",
  "gene": "UniProtKB:P08588",
  "gene_symbol": "ADRB1"
}